{
  "gene_name": "DNA-directed RNA polymerases I, II, and III subunit RPABC5",
  "gene": "UniProtKB:P62875",
  "term_id": "GO:0005666",
  "gene_symbol": "POLR2L",
  "term_label": "RNA polymerase III complex"
}